{
  "gene_name": "DNA-binding protein SMUBP-2",
  "gene_symbol": "IGHMBP2",
  "gene": "UniProtKB:P38935",
  "term_id": "GO:0006974",
  "term_label": "DNA damage response"
}